hypothalamus cell migration [GO:0021855] (biological process) Definition: The directed movement of a cell into the hypothalamus region of the forebrain. Relationships: is_a cell migration [GO:0016477]; is part of hypothalamus development [GO:0021854] Subtypes: hypothalamic tangential migration using cell-axon interactions [GO:0021856] Sources: GOC:cls, GOC:dgh, GOC:dph, GOC:jid, GO_REF:0000021